{
  "gene_name": "Short-chain dehydrogenase_reductase family 9C member 7",
  "term_label": "retinol metabolic process",
  "gene_symbol": "SDR9C7",
  "gene": "UniProtKB:Q8NEX9",
  "term_id": "GO:0042572"
}